{
  "term_label": "nucleus",
  "gene_name": "Nucleosome assembly protein 1-like 4",
  "term_id": "GO:0005634",
  "gene": "UniProtKB:Q99733",
  "gene_symbol": "NAP1L4"
}